phosphatidylinositol 3-kinase complex, class IA [GO:0005943] (cellular component) Relationships: is a type of GO:0097651 Also known as: 1-phosphatidylinositol-4-phosphate 3-kinase, class IA complex, 1-phosphatidylinositol-4-phosphate kinase, class IA complex, class IA PI3K complex, phosphoinositide 3-kinase complex, class IA References: PMID:9255069, PMID:9759495 Definition: A class I phosphatidylinositol 3-kinase complex that possesses 1-phosphatidylinositol-4-phosphate 3-kinase activity; comprises a catalytic class IA phosphoinositide 3-kinase (PI3K) subunit and an associated SH2 domain-containing regulatory subunit that is a member of a family of related proteins often called p85 proteins. Through the interaction with the SH2-containing adaptor subunits, Class IA PI3K catalytic subunits are linked to tyrosine kinase signaling pathways.